terminal button organization [GO:0072553] (biological process) Definition: A process that is carried out at the cellular level which results in the assembly, arrangement of constituent parts, or disassembly of a terminal button. A terminal button is the terminal inflated portion of the axon, containing the specialized apparatus necessary to release neurotransmitters. Sources: GOC:BHF, GOC:mah Also known as: bouton organization, presynaptic bouton organization, synaptic bouton organization, terminal bouton organization, terminal button organisation Relationships: is a type of presynapse organization [GO:0099172] Regulation: negatively regulated by negative regulation of terminal button organization [GO:1901613]; positively regulated by GO:1901614; regulated by regulation of terminal button organization [GO:2000331]